{
  "gene": "UniProtKB:Q969P5",
  "term_id": "GO:0016567",
  "gene_name": "F-box only protein 32",
  "gene_symbol": "FBXO32",
  "term_label": "protein ubiquitination"
}